removal of superoxide radicals [GO:0019430] (biological process) Regulation: negatively regulated by GO:1904832; RO_0002213 by positive regulation of removal of superoxide radicals [GO:1904833]; regulated by regulation of removal of superoxide radicals [GO:2000121] Also known as: cellular detoxification of superoxide radicals, removal of O2-, removal of oxygen free radicals Relationships: is a type of GO:0006801; is_a GO:0098869; is part of GO:0071451 Definition: Any process, acting at the cellular level, involved in removing superoxide radicals (O2-) from a cell or organism, e.g. by conversion to dioxygen (O2) and hydrogen peroxide (H2O2). Sources: GOC:jl